{
  "gene_symbol": "GBX1",
  "gene": "UniProtKB:Q14549",
  "term_id": "GO:0051960",
  "gene_name": "Homeobox protein GBX-1",
  "term_label": "regulation of nervous system development"
}